extraembryonic membrane development [GO:1903867] (biological process) Definition: The process whose specific outcome is the progression of an extraembryonic membrane over time, from its formation to the mature structure. Sources: GOC:TermGenie, GO_REF:0000094, ISBN:0073040584 Relationships: is a type of anatomical structure development [GO:0048856] Subtypes: chorion development [GO:0060717], GO:1905069